{
  "gene_symbol": "PAFAH1B2",
  "term_id": "GO:0003847",
  "gene_name": "Platelet-activating factor acetylhydrolase IB subunit alpha2",
  "term_label": "1-alkyl-2-acetylglycerophosphocholine esterase activity",
  "gene": "UniProtKB:P68402"
}